positive regulation of 1-phosphatidyl-1D-myo-inositol 4,5-bisphosphate catabolic process [GO:1902643] (biological process) References: PMID:22562153 Sources: GOC:TermGenie, GOC:di, GO_REF:0000058 Definition: Any process that activates or increases the frequency, rate or extent of 1-phosphatidyl-1D-myo-inositol 4,5-bisphosphate catabolic process. Also known as: positive regulation of 1-phosphatidyl-1D-myo-inositol 4,5-bisphosphate breakdown, positive regulation of 1-phosphatidyl-1D-myo-inositol 4,5-bisphosphate catabolism, positive regulation of 1-phosphatidyl-1D-myo-inositol 4,5-bisphosphate degradation, up regulation of 1-phosphatidyl-1D-myo-inositol 4,5-bisphosphate breakdown, up regulation of 1-phosphatidyl-1D-myo-inositol 4,5-bisphosphate catabolic process, up regulation of 1-phosphatidyl-1D-myo-inositol 4,5-bisphosphate catabolism, up regulation of 1-phosphatidyl-1D-myo-inositol 4,5-bisphosphate degradation, up-regulation of 1-phosphatidyl-1D-myo-inositol 4,5-bisphosphate breakdown, up-regulation of 1-phosphatidyl-1D-myo-inositol 4,5-bisphosphate catabolic process, up-regulation of 1-phosphatidyl-1D-myo-inositol 4,5-bisphosphate catabolism, up-regulation of 1-phosphatidyl-1D-myo-inositol 4,5-bisphosphate degradation, upregulation of 1-phosphatidyl-1D-myo-inositol 4,5-bisphosphate breakdown, upregulation of 1-phosphatidyl-1D-myo-inositol 4,5-bisphosphate catabolic process, upregulation of 1-phosphatidyl-1D-myo-inositol 4,5-bisphosphate catabolism, upregulation of 1-phosphatidyl-1D-myo-inositol 4,5-bisphosphate degradation, activation of 1-phosphatidyl-1D-myo-inositol 4,5-bisphosphate breakdown, activation of 1-phosphatidyl-1D-myo-inositol 4,5-bisphosphate catabolic process, activation of 1-phosphatidyl-1D-myo-inositol 4,5-bisphosphate catabolism, activation of 1-phosphatidyl-1D-myo-inositol 4,5-bisphosphate degradation Relationships: is a type of positive regulation of phospholipid catabolic process [GO:0060697]; is a type of regulation of 1-phosphatidyl-1D-myo-inositol 4,5-bisphosphate catabolic process [GO:1902641]; positively regulates GO:1902634